{
  "term_id": "GO:0045944",
  "term_label": "positive regulation of transcription by RNA polymerase II",
  "gene": "UniProtKB:P61371",
  "gene_symbol": "ISL1",
  "gene_name": "Insulin gene enhancer protein ISL-1"
}